{
  "gene_symbol": "ATPAF1",
  "term_label": "mitochondrial proton-transporting ATP synthase complex assembly",
  "gene_name": "ATP synthase mitochondrial F1 complex assembly factor 1",
  "gene": "UniProtKB:Q5TC12",
  "term_id": "GO:0033615"
}